{
  "gene": "UniProtKB:P19793",
  "gene_symbol": "RXRA",
  "term_label": "retinoic acid-responsive element binding",
  "term_id": "GO:0044323",
  "gene_name": "Retinoic acid receptor RXR-alpha"
}